{
  "gene_name": "E3 ubiquitin ligase TRAF3IP2",
  "term_label": "Unknown molecular function",
  "gene_symbol": "TRAF3IP2",
  "term_id": "UNKNOWN:0001",
  "gene": "UniProtKB:O43734"
}